{
  "gene_symbol": "OR13C9",
  "term_label": "olfactory receptor activity",
  "gene_name": "Olfactory receptor 13C9",
  "gene": "UniProtKB:Q8NGT0",
  "term_id": "GO:0004984"
}